cardiac ventricle morphogenesis [GO:0003208] (biological process) Sources: GOC:mtg_heart Subtypes: cardiac left ventricle morphogenesis [GO:0003214], GO:0003215 Definition: The process in which the cardiac ventricle is generated and organized. A cardiac ventricle receives blood from a cardiac atrium and pumps it out of the heart. Relationships: is a type of GO:0003206; is part of GO:0003231